{
  "gene_name": "Serine_threonine-protein phosphatase 2A activator",
  "term_label": "peptidyl-prolyl cis-trans isomerase activity",
  "gene": "UniProtKB:Q15257",
  "term_id": "GO:0003755",
  "gene_symbol": "PTPA"
}